regulation of sterol import [GO:2000909] (biological process) Sources: GOC:obol Definition: Any process that modulates the frequency, rate or extent of sterol import. Relationships: is a type of regulation of sterol transport [GO:0032371]; regulates sterol import [GO:0035376] Subtypes: negative regulation of sterol import [GO:2000910], positive regulation of sterol import [GO:2000911] Also known as: regulation of sterol influx, regulation of sterol uptake